regulation of iodide transmembrane transport [GO:1904212] (biological process) Definition: Any process that modulates the frequency, rate or extent of iodide transmembrane transport. Relationships: is a type of regulation of monoatomic anion transmembrane transport [GO:1903959]; is a type of regulation of iodide transport [GO:1904201]; regulates GO:1904200 Subtypes: negative regulation of iodide transmembrane transport [GO:1904213], positive regulation of iodide transmembrane transport [GO:1904214] References: PMID:20392814 Sources: GOC:TermGenie, GO_REF:0000058